{
  "gene": "UniProtKB:Q9H081",
  "gene_symbol": "MIS12",
  "term_label": "Unknown molecular function",
  "gene_name": "Protein MIS12 homolog",
  "term_id": "UNKNOWN:0001"
}